11-cis-retinyl-palmitate hydrolase activity [GO:0047520] (molecular function) Definition: Catalysis of the reaction: 11-cis-retinyl palmitate + H2O = 11-cis-retinol + H+ + palmitate. Also known as: 11-cis-retinol palmitate esterase activity, 11-cis-retinyl-palmitate acylhydrolase activity, RPH Relationships: is a type of GO:0052689; is part of retinol metabolic process [GO:0042572] Sources: EC:3.1.1.63, RHEA:19697